{
  "gene_name": "Aquaporin-7",
  "gene": "UniProtKB:O14520",
  "term_label": "water transport",
  "term_id": "GO:0006833",
  "gene_symbol": "AQP7"
}